{
  "gene_symbol": "ZP4",
  "gene": "UniProtKB:Q12836",
  "term_label": "egg coat",
  "term_id": "GO:0035805",
  "gene_name": "Zona pellucida sperm-binding protein 4"
}